amyloplast envelope [GO:0033096] (cellular component) Sources: GOC:mah Relationships: is a type of GO:0009526; is part of amyloplast [GO:0009501] Definition: The double lipid bilayer enclosing the amyloplast and separating its contents from the rest of the cytoplasm; includes the intermembrane space.